{
  "term_label": "plasma membrane",
  "gene": "UniProtKB:Q7RTX9",
  "term_id": "GO:0005886",
  "gene_symbol": "SLC16A14",
  "gene_name": "Monocarboxylate transporter 14"
}